{
  "gene": "UniProtKB:Q5VZ18",
  "gene_symbol": "SHE",
  "gene_name": "SH2 domain-containing adapter protein E",
  "term_label": "Unknown cellular component",
  "term_id": "UNKNOWN:0003"
}